{
  "term_id": "GO:0005737",
  "gene": "UniProtKB:Q9Y446",
  "term_label": "cytoplasm",
  "gene_symbol": "PKP3",
  "gene_name": "Plakophilin-3"
}